{
  "gene_name": "MIF4G domain-containing protein",
  "gene_symbol": "MIF4GD",
  "term_id": "GO:0006446",
  "term_label": "regulation of translational initiation",
  "gene": "UniProtKB:A9UHW6"
}